positive regulation of snRNA transcription by RNA polymerase II [GO:1905382] (biological process) Relationships: is a type of GO:0045944; is a type of regulation of snRNA transcription by RNA polymerase II [GO:1905380]; positively regulates snRNA transcription by RNA polymerase II [GO:0042795] Definition: Any process that activates or increases the frequency, rate or extent of snRNA transcription mediated by RNA polymerase II. Note: An example of this is GTF2A1 in human (UniProt symbol P52655) in PMID:10022900 (inferred from direct assay). References: PMID:10022900 Sources: GOC:TermGenie, GOC:bhm, GO_REF:0000058 Also known as: positive regulation of snRNA transcription from Pol II promoter, positive regulation of snRNA transcription from RNA polymerase II promoter, up regulation of snRNA transcription from Pol II promoter, up regulation of snRNA transcription from RNA polymerase II promoter, up-regulation of snRNA transcription from Pol II promoter, up-regulation of snRNA transcription from RNA polymerase II promoter, upregulation of snRNA transcription from Pol II promoter, upregulation of snRNA transcription from RNA polymerase II promoter, activation of snRNA transcription from Pol II promoter, activation of snRNA transcription from RNA polymerase II promoter